excitatory postsynaptic potential [GO:0060079] (biological process) Also known as: regulation of excitatory post-synaptic membrane potential, regulation of EPSP Sources: GOC:dph, GOC:ef Definition: A process that leads to a temporary increase in postsynaptic potential due to the flow of positively charged ions into the postsynaptic cell. The flow of ions that causes an EPSP is an excitatory postsynaptic current (EPSC) and makes it easier for the neuron to fire an action potential. Relationships: is a type of GO:0060078; is part of GO:0099565 Subtypes: mini excitatory postsynaptic potential [GO:0098816], evoked excitatory postsynaptic potential [GO:0098817] Regulation: negatively regulated by negative regulation of excitatory postsynaptic potential [GO:0090394]; regulated by modulation of excitatory postsynaptic potential [GO:0098815]; positively regulated by GO:2000463